{
  "gene_name": "Zinc finger protein PLAGL1",
  "gene": "UniProtKB:Q9UM63",
  "term_label": "DNA-binding transcription repressor activity, RNA polymerase II-specific",
  "term_id": "GO:0001227",
  "gene_symbol": "PLAGL1"
}